negative regulation of osteoblast differentiation [GO:0045668] (biological process) Relationships: is a type of negative regulation of cell differentiation [GO:0045596]; is a type of regulation of osteoblast differentiation [GO:0045667]; negatively regulates osteoblast differentiation [GO:0001649] Also known as: down regulation of osteoblast differentiation, down-regulation of osteoblast differentiation, downregulation of osteoblast differentiation, inhibition of osteoblast differentiation Sources: GOC:go_curators Definition: Any process that stops, prevents, or reduces the frequency, rate or extent of osteoblast differentiation.